{
  "term_label": "Unknown cellular component",
  "gene_symbol": "AKT2",
  "gene_name": "RAC-beta serine_threonine-protein kinase",
  "gene": "UniProtKB:P31751",
  "term_id": "UNKNOWN:0003"
}